{
  "term_id": "GO:0006884",
  "gene_symbol": "SLC12A4",
  "gene_name": "Solute carrier family 12 member 4",
  "gene": "UniProtKB:Q9UP95",
  "term_label": "cell volume homeostasis"
}